{
  "gene_symbol": "CGB1",
  "term_id": "GO:0007186",
  "gene": "UniProtKB:A6NKQ9",
  "gene_name": "Choriogonadotropin subunit beta variant 1",
  "term_label": "G protein-coupled receptor signaling pathway"
}